cell integrity MAPK cascade [GO:0000196] (biological process) Regulation: regulated by regulation of cell integrity MAPK cascade [GO:1903137]; RO_0002212 by negative regulation of cell integrity MAPK cascade [GO:1903138]; positively regulated by positive regulation of cell integrity MAPK cascade [GO:1903139] Sources: GOC:vw Definition: A MAPK cascade that specifically ensures the maintenance and regulation of cellular structure in response to external signals, including plasma membrane stretching or cell wall alteration, to coordinate cellular responses such as growth, differentiation, and stress adaptation, thereby preserving cell integrity. Contains the  SLT2 (S.cerevisiae)/Pmk1 (S.pombe) MAP kinase or orthologs. Relationships: is a type of GO:0051403 Also known as: cell integrity MAPK pathway, Mpk1 cascade, PMK1-MAPK signal transduction pathway, Pmk1 MAPK cell integrity signaling, Pmk1 mitogen-activated protein kinase (MAPK) cell integrity pathway, Slt2 cascade, cell wall integrity MAPK cascade, CWI pathway